{
  "term_id": "GO:0005634",
  "gene_name": "Zinc finger protein 385C",
  "gene_symbol": "ZNF385C",
  "gene": "UniProtKB:Q66K41",
  "term_label": "nucleus"
}